{
  "gene": "UniProtKB:P01568",
  "gene_symbol": "IFNA21",
  "term_label": "type I interferon receptor binding",
  "term_id": "GO:0005132",
  "gene_name": "Interferon alpha-21"
}